{
  "gene_name": "Elongation factor 1-alpha 2",
  "term_id": "GO:0006414",
  "term_label": "translational elongation",
  "gene": "UniProtKB:Q05639",
  "gene_symbol": "EEF1A2"
}